{
  "gene_name": "Ankyrin repeat domain-containing protein 60",
  "term_label": "Unknown cellular component",
  "term_id": "UNKNOWN:0003",
  "gene_symbol": "ANKRD60",
  "gene": "UniProtKB:Q9BZ19"
}